{
  "term_id": "GO:0003729",
  "gene_symbol": "TEX13A",
  "gene": "UniProtKB:Q9BXU3",
  "gene_name": "Testis-expressed protein 13A",
  "term_label": "mRNA binding"
}